protein O-linked glycosylation [GO:0006493] (biological process) Definition: A glycoprotein biosynthetic process starting with the covalent linkage of carbohydrate or carbohydrate derivative unit via a glycosidic bond to the oxygen atom of a serine, threonine, hydroxylysine, hydroxyproline or tyrosine side chain in a protein, which can be further elongated with the sequential addition of sugar units resulting in the formation of a protein O-linked glycan. References: PMID:33775405 Subtypes: protein O-linked glycosylation via N-acetyl-galactosamine [GO:0016266], protein O-linked glycosylation via mannose [GO:0035269], protein O-linked glycosylation via fucose [GO:0036066], protein O-linked glycosylation via glucose [GO:0180059], protein O-linked glycosylation via galactose [GO:0180062], protein O-linked glycosylation via arabinose [GO:0180063], GO:0180064 Also known as: protein amino acid O-linked glycosylation Regulation: regulated by GO:1904098; negatively regulated by negative regulation of protein O-linked glycosylation [GO:1904099]; positively regulated by positive regulation of protein O-linked glycosylation [GO:1904100] Relationships: is a type of glycoprotein biosynthetic process [GO:0009101]